{
  "gene_name": "RecQ-mediated genome instability protein 2",
  "gene_symbol": "RMI2",
  "gene": "UniProtKB:Q96E14",
  "term_id": "GO:0016607",
  "term_label": "nuclear speck"
}